{
  "gene": "UniProtKB:O00750",
  "term_label": "1-phosphatidylinositol-3-kinase activity",
  "term_id": "GO:0016303",
  "gene_name": "Phosphatidylinositol 4-phosphate 3-kinase C2 domain-containing subunit beta",
  "gene_symbol": "PIK3C2B"
}